inositol hexakisphosphate 3-kinase activity [GO:0052724] (molecular function) Relationships: is a type of inositol hexakisphosphate kinase activity [GO:0000828] Definition: Catalysis of the reaction: ATP + 1D-myo-inositol hexakisphosphate = ADP + 3-diphospho-1D-myo-inositol (1,2,4,5,6)pentakisphosphate. References: PMID:18981179 Sources: MetaCyc:RXN-10971